{
  "term_label": "monoatomic cation transmembrane transport",
  "gene_symbol": "TRPM6",
  "gene_name": "Transient receptor potential cation channel subfamily M member 6",
  "term_id": "GO:0098655",
  "gene": "UniProtKB:Q9BX84"
}